{
  "gene": "UniProtKB:P01871",
  "term_id": "UNKNOWN:0001",
  "gene_symbol": "IGHM",
  "term_label": "Unknown molecular function",
  "gene_name": "Immunoglobulin heavy constant mu"
}